{
  "term_label": "Unknown molecular function",
  "gene_symbol": "AVL9",
  "term_id": "UNKNOWN:0001",
  "gene_name": "Late secretory pathway protein AVL9 homolog",
  "gene": "UniProtKB:Q8NBF6"
}